{
  "gene": "UniProtKB:Q14008",
  "term_label": "centrosome",
  "gene_name": "Cytoskeleton-associated protein 5",
  "term_id": "GO:0005813",
  "gene_symbol": "CKAP5"
}